{
  "gene": "UniProtKB:Q96QE2",
  "gene_symbol": "SLC2A13",
  "term_id": "GO:0055085",
  "gene_name": "Proton myo-inositol cotransporter",
  "term_label": "transmembrane transport"
}